acetylsalicylate deacetylase activity [GO:0047610] (MF) Also known as: acetylsalicylate O-acetylhydrolase activity, acetylsalicylic acid esterase activity, aspirin esterase activity, aspirin hydrolase activity Definition: Catalysis of the reaction: acetylsalicylate + H2O = acetate + H+ + salicylate. Relationships: is a type of deacetylase activity [GO:0019213]; is a type of GO:0052689 Sources: EC:3.1.1.55, RHEA:11752